regulation of endodermal cell differentiation [GO:1903224] (biological process) Definition: Any process that modulates the frequency, rate or extent of endodermal cell differentiation. Relationships: is a type of GO:0045595; regulates endodermal cell differentiation [GO:0035987] Also known as: regulation of endoderm cell differentiation Subtypes: regulation of endodermal cell fate specification [GO:0042663], GO:1903225, positive regulation of endodermal cell differentiation [GO:1903226] References: PMID:23154389 Sources: GOC:TermGenie, GOC:als, GO_REF:0000058